{
  "gene_name": "CDC42 small effector protein 1",
  "gene": "UniProtKB:Q9NRR8",
  "term_id": "UNKNOWN:0001",
  "gene_symbol": "CDC42SE1",
  "term_label": "Unknown molecular function"
}